{
  "term_label": "cilium assembly",
  "gene": "UniProtKB:Q2MV58",
  "gene_symbol": "TCTN1",
  "term_id": "GO:0060271",
  "gene_name": "Tectonic-1"
}